regulation of interleukin-2 production [GO:0032663] (biological process) Subtypes: negative regulation of interleukin-2 production [GO:0032703], positive regulation of interleukin-2 production [GO:0032743] Definition: Any process that modulates the frequency, rate, or extent of interleukin-2 production. Sources: GOC:mah Relationships: is a type of regulation of cytokine production [GO:0001817]; regulates GO:0032623 Also known as: regulation of IL-2 production, regulation of interleukin-2 biosynthetic process, regulation of interleukin-2 secretion